{
  "term_label": "Unknown molecular function",
  "term_id": "UNKNOWN:0001",
  "gene": "UniProtKB:Q24JP5",
  "gene_name": "Transmembrane protein 132A",
  "gene_symbol": "TMEM132A"
}